{
  "gene_name": "BTB_POZ domain-containing adapter for CUL3-mediated RhoA degradation protein 1",
  "term_label": "proteasome-mediated ubiquitin-dependent protein catabolic process",
  "gene_symbol": "KCTD13",
  "term_id": "GO:0043161",
  "gene": "UniProtKB:Q8WZ19"
}